purinergic nucleotide receptor signaling pathway [GO:0035590] (biological process) Relationships: is a type of cell surface receptor signaling pathway [GO:0007166] References: PMID:9755289 Sources: GOC:BHF Also known as: purinergic nucleotide receptor signalling pathway, P2 receptor signaling pathway, purinergic receptor signaling pathway, purinergic receptor signalling pathway, purinoceptor signaling pathway Subtypes: GO:0035588, G protein-coupled purinergic nucleotide receptor signaling pathway [GO:0035589] Definition: The series of molecular signals initiated by an extracellular purine nucleotide binding to its receptor, and ending with the regulation of a downstream cellular process, e.g. transcription.